{
  "term_label": "kynurenine-oxoglutarate transaminase activity",
  "gene_symbol": "KYAT1",
  "gene": "UniProtKB:Q16773",
  "term_id": "GO:0016212",
  "gene_name": "Kynurenine--oxoglutarate transaminase 1"
}